{
  "term_id": "UNKNOWN:0002",
  "term_label": "Unknown biological process",
  "gene": "UniProtKB:Q6ZTI0",
  "gene_name": "Putative uncharacterized protein FLJ44636",
  "gene_symbol": "Q6ZTI0"
}